{
  "term_label": "Unknown cellular component",
  "gene": "UniProtKB:P43251",
  "gene_name": "Biotinidase",
  "gene_symbol": "BTD",
  "term_id": "UNKNOWN:0003"
}